{
  "gene": "UniProtKB:Q8WWZ4",
  "term_id": "GO:0006869",
  "term_label": "lipid transport",
  "gene_name": "ATP-binding cassette sub-family A member 10",
  "gene_symbol": "ABCA10"
}